{
  "gene_name": "Glucose-dependent insulinotropic receptor",
  "gene": "UniProtKB:Q8TDV5",
  "term_label": "phosphatidylcholine binding",
  "term_id": "GO:0031210",
  "gene_symbol": "GPR119"
}